{
  "gene_symbol": "CFAP100",
  "gene": "UniProtKB:Q494V2",
  "term_id": "UNKNOWN:0002",
  "term_label": "Unknown biological process",
  "gene_name": "Cilia- and flagella-associated protein 100"
}